{
  "gene_symbol": "CSF2RB",
  "term_id": "GO:0038157",
  "gene": "UniProtKB:P32927",
  "gene_name": "Cytokine receptor common subunit beta",
  "term_label": "granulocyte-macrophage colony-stimulating factor signaling pathway"
}